CUU codon-amino acid adaptor activity [GO:0033417] (molecular function) Also known as: CTT codon-amino acid adaptor activity, leucine tRNA Note: Note that in the standard genetic code, CTT codes for leucine. Relationships: is a type of triplet codon-amino acid adaptor activity [GO:0030533] Definition: A triplet codon-amino acid adaptor activity that recognizes a CUU codon. Sources: GOC:mah